{
  "gene_symbol": "PPP1R3C",
  "gene": "UniProtKB:Q9UQK1",
  "term_label": "glycogen binding",
  "term_id": "GO:2001069",
  "gene_name": "Protein phosphatase 1 regulatory subunit 3C"
}